acetate ester metabolic process involved in fermentation [GO:1901089] (biological process) Definition: Any acetate ester metabolic process that is involved in fermentation. Relationships: is_a fermentation [GO:0006113] Also known as: acetate ester metabolic process during fermentation Sources: GOC:TermGenie, GOC:sgd_curators